{
  "gene_symbol": "KARS1",
  "gene_name": "Lysine--tRNA ligase",
  "gene": "UniProtKB:Q15046",
  "term_label": "tRNA binding",
  "term_id": "GO:0000049"
}